regulation of translation at synapse, modulating synaptic transmission [GO:0099547] (biological process) Relationships: is a type of modulation of chemical synaptic transmission [GO:0050804]; is_a regulation of translation at synapse [GO:0140243] Note: Note that this term was created for the SynGO project, and will be obsoleted when the SynGO annotations are made in Noctua. Sources: GOC:dos Definition: Any process that modulates synaptic transmission by regulating translation occurring at the synapse. Subtypes: regulation of translation at presynapse, modulating synaptic transmission [GO:0099577], regulation of translation at postsynapse, modulating synaptic transmission [GO:0099578]